{
  "gene_name": "GTP-binding protein 1",
  "gene": "UniProtKB:O00178",
  "gene_symbol": "GTPBP1",
  "term_id": "GO:0006414",
  "term_label": "translational elongation"
}